response to bisphenol A [GO:1903925] (biological process) Definition: Any process that results in a change in state or activity of a cell or an organism (in terms of movement, secretion, enzyme production, gene expression, etc.) as a result of a bisphenol A stimulus. References: PMID:22957036 Sources: GOC:TermGenie, GO_REF:0000071 Relationships: is a type of response to oxygen-containing compound [GO:1901700] Subtypes: cellular response to bisphenol A [GO:1903926]